{
  "term_label": "[protein]-3-O-(N-acetyl-D-glucosaminyl)-L-serine/L-threonine O-N-acetyl-alpha-D-glucosaminase activity",
  "term_id": "GO:0102571",
  "gene_symbol": "OGA",
  "gene_name": "Protein O-GlcNAcase",
  "gene": "UniProtKB:O60502"
}